{
  "gene_symbol": "GSDMC",
  "term_label": "pyroptotic inflammatory response",
  "gene": "UniProtKB:Q9BYG8",
  "gene_name": "Gasdermin-C",
  "term_id": "GO:0070269"
}